negative regulation of translation in response to oxidative stress [GO:0032938] (biological process) Relationships: is a type of negative regulation of translational initiation in response to stress [GO:0032057]; is a type of GO:0043556; is a type of regulation of translational initiation in response to stress [GO:0043558] Definition: Any process that stops, prevents, or reduces the frequency, rate or extent of translation as a result of oxidative stress, a state often resulting from exposure to high levels of reactive oxygen species, e.g. superoxide anions, hydrogen peroxide (H2O2), and hydroxyl radicals. Sources: GOC:mah